{
  "gene_name": "Leucine-rich repeat and IQ domain-containing protein 1",
  "gene": "UniProtKB:Q96JM4",
  "term_id": "GO:0015630",
  "gene_symbol": "LRRIQ1",
  "term_label": "microtubule cytoskeleton"
}